{
  "gene": "UniProtKB:O75530",
  "gene_symbol": "EED",
  "gene_name": "Polycomb protein EED",
  "term_id": "GO:0031491",
  "term_label": "nucleosome binding"
}